melanin biosynthetic process [GO:0042438] (biological process) Regulation: regulated by regulation of melanin biosynthetic process [GO:0048021]; negatively regulated by negative regulation of melanin biosynthetic process [GO:0048022]; positively regulated by positive regulation of melanin biosynthetic process [GO:0048023] Subtypes: melanin biosynthetic process from tyrosine [GO:0006583], 1,8-dihydroxynaphthalene-melanin biosynthetic process [GO:0140614] Sources: GOC:curators Definition: The chemical reactions and pathways resulting in the formation of melanins, pigments largely of animal origin. High molecular weight polymers of indole quinone, they are irregular polymeric structures and are divided into three groups: allomelanins in the plant kingdom and eumelanins and phaeomelanins in the animal kingdom. Also known as: melanin anabolism, melanin biosynthesis, melanin formation, melanin synthesis Relationships: is a type of melanin metabolic process [GO:0006582]; is a type of secondary metabolite biosynthetic process [GO:0044550]; is a type of pigment biosynthetic process [GO:0046148]; is_a phenol-containing compound biosynthetic process [GO:0046189]